mesenchymal cell differentiation [GO:0048762] (biological process) Definition: The process in which a relatively unspecialized cell acquires specialized features of a mesenchymal cell. A mesenchymal cell is a loosely associated cell that is part of the connective tissue in an organism. Mesenchymal cells give rise to more mature connective tissue cell types. Sources: GOC:dph, GOC:jid Relationships: is a type of cell differentiation [GO:0030154]; is part of mesenchyme development [GO:0060485] Subtypes: epithelial to mesenchymal transition [GO:0001837], neural crest cell differentiation [GO:0014033], mesenchymal cell differentiation involved in mammary gland development [GO:0060610], mesenchymal cell differentiation involved in salivary gland development [GO:0060692], mesenchymal cell differentiation involved in lung development [GO:0060915], cardiac endothelial to mesenchymal transition [GO:0140074], mesenchymal cell differentiation involved in bone development [GO:1901706], mesenchymal cell differentiation involved in renal system development [GO:2001012]